{
  "gene_symbol": "NDFIP2",
  "term_id": "UNKNOWN:0001",
  "gene_name": "NEDD4 family-interacting protein 2",
  "gene": "UniProtKB:Q9NV92",
  "term_label": "Unknown molecular function"
}